{
  "gene_symbol": "PFKL",
  "gene_name": "ATP-dependent 6-phosphofructokinase, liver type",
  "term_id": "GO:0070095",
  "term_label": "fructose-6-phosphate binding",
  "gene": "UniProtKB:P17858"
}